rhombomere 5 development [GO:0021571] (biological process) Definition: The process whose specific outcome is the progression of rhombomere 5 over time, from its formation to the mature structure. Rhombomeres are transverse segments of the developing rhombencephalon. Rhombomeres are lineage restricted, express different genes from one another, and adopt different developmental fates. Rhombomeres are numbered in anterior to posterior order. Sources: GOC:cls, GOC:curators, GOC:dgh, GOC:dph, GOC:jid Relationships: is a type of GO:0021546